positive regulation of antigen processing and presentation of peptide antigen via MHC class Ib [GO:0002597] (BP) Definition: Any process that activates or increases the frequency, rate, or extent of antigen processing and presentation of peptide antigen via MHC class Ib. Sources: GOC:add Also known as: positive regulation of peptide antigen processing and presentation via MHC class Ib, up regulation of antigen processing and presentation of peptide antigen via MHC class Ib, up-regulation of antigen processing and presentation of peptide antigen via MHC class Ib, upregulation of antigen processing and presentation of peptide antigen via MHC class Ib, activation of antigen processing and presentation of peptide antigen via MHC class Ib, stimulation of antigen processing and presentation of peptide antigen via MHC class Ib Relationships: is a type of positive regulation of antigen processing and presentation of peptide antigen [GO:0002585]; is a type of positive regulation of antigen processing and presentation via MHC class Ib [GO:0002594]; is a type of regulation of antigen processing and presentation of peptide antigen via MHC class Ib [GO:0002595]; positively regulates antigen processing and presentation of peptide antigen via MHC class Ib [GO:0002428]